{
  "term_label": "ubiquitin-protein transferase activity",
  "gene": "UniProtKB:Q63HN8",
  "gene_name": "E3 ubiquitin-protein ligase RNF213",
  "term_id": "GO:0004842",
  "gene_symbol": "RNF213"
}